{
  "term_label": "maintenance of centrosome location",
  "gene_symbol": "TBCCD1",
  "gene": "UniProtKB:Q9NVR7",
  "gene_name": "TBCC domain-containing protein 1",
  "term_id": "GO:0051661"
}